regulation of NK T cell differentiation [GO:0051136] (biological process) References: PMID:12154375, PMID:9133426 Sources: ISBN:0781735149 Note: Note that immunologists typically use the word 'development' to refer to cells of B or T cell lineages undergoing the process that GO describes as 'cell differentiation'. Relationships: is_a regulation of alpha-beta T cell differentiation [GO:0046637]; regulates GO:0001865 Definition: Any process that modulates the frequency, rate or extent of natural killer T cell differentiation. Subtypes: negative regulation of NK T cell differentiation [GO:0051137], GO:0051138 Also known as: regulation of NK T lymphocyte differentiation, regulation of NK T-cell differentiation, regulation of NK T-lymphocyte differentiation, regulation of NKT cell differentiation, regulation of NT cell differentiation, regulation of natural T cell differentiation, regulation of natural killer T cell differentiation, regulation of NK T cell development